{
  "gene": "UniProtKB:P34981",
  "term_id": "GO:0004997",
  "gene_symbol": "TRHR",
  "gene_name": "Thyrotropin-releasing hormone receptor",
  "term_label": "thyrotropin-releasing hormone receptor activity"
}